{
  "gene_name": "Peptidyl-prolyl cis-trans isomerase C",
  "term_id": "GO:0003755",
  "gene_symbol": "PPIC",
  "term_label": "peptidyl-prolyl cis-trans isomerase activity",
  "gene": "UniProtKB:P45877"
}